{
  "gene": "UniProtKB:Q9H0H0",
  "term_label": "integrator complex",
  "gene_symbol": "INTS2",
  "gene_name": "Integrator complex subunit 2",
  "term_id": "GO:0032039"
}